{
  "gene_name": "Peroxiredoxin-1",
  "gene_symbol": "PRDX1",
  "term_id": "GO:0042744",
  "gene": "UniProtKB:Q06830",
  "term_label": "hydrogen peroxide catabolic process"
}